regulation of endothelial cell activation [GO:1904987] (biological process) References: PMID:24255059 Sources: GOC:BHF, GOC:BHF_miRNA, GOC:TermGenie, GOC:bc, GO_REF:0000058 Subtypes: negative regulation of endothelial cell activation [GO:1904988], positive regulation of endothelial cell activation [GO:1904989] Definition: Any process that modulates the frequency, rate or extent of endothelial cell activation. Relationships: is a type of GO:0050865; regulates endothelial cell activation [GO:0042118]